{
  "term_label": "retrograde transport, endosome to Golgi",
  "gene_name": "TBC1 domain family member 23",
  "term_id": "GO:0042147",
  "gene": "UniProtKB:Q9NUY8",
  "gene_symbol": "TBC1D23"
}